{
  "term_label": "detection of chemical stimulus involved in sensory perception of smell",
  "gene": "UniProtKB:Q8NH19",
  "gene_symbol": "OR10AG1",
  "gene_name": "Olfactory receptor 10AG1",
  "term_id": "GO:0050911"
}